negative regulation of gene expression via chromosomal CpG island methylation [GO:0044027] (biological process) References: PMID:11898023 Sources: Wikipedia:Cpg_island Relationships: is a type of negative regulation of gene expression, epigenetic [GO:0045814] Also known as: maintenance of DNA methylation, DNA hypermethylation of CpG island, epigenetic regulation of gene expression via CpG island hypermethylation, hypermethylation of CpG island, negative regulation of gene expression via CpG island hypermethylation, negative regulation of gene expression via chromosomal CpG dinucleotide methylation, negative regulation of gene expression via chromosomal DNA cytosine methylation, DNA hypermethylation of CG island, negative regulation of gene expression via CpG island methylation, negative regulation of gene expression via chromosomal CG dinucleotide methylation Definition: An epigenetic gene regulation mechanism that negatively regulates gene expression by methylation of cytosine residues in chromosomal CpG islands. CpG islands are genomic regions that contain a high frequency of the CG dinucleotide associated with the transcription start site of genes.